cell proliferation in dorsal spinal cord [GO:0010456] (biological process) Definition: The multiplication or reproduction of cells, resulting in the expansion of the dorsal spinal cord cell population. Sources: GOC:dph, GOC:tb Relationships: is a type of GO:0061351 Regulation: regulated by regulation of cell proliferation in dorsal spinal cord [GO:0021921]; negatively regulated by GO:1902832; positively regulated by positive regulation of cell proliferation in dorsal spinal cord [GO:1902833]